{
  "term_id": "GO:0006357",
  "gene_symbol": "KLF5",
  "gene_name": "Krueppel-like factor 5",
  "gene": "UniProtKB:Q13887",
  "term_label": "regulation of transcription by RNA polymerase II"
}